{
  "gene": "UniProtKB:P20783",
  "term_label": "nerve growth factor signaling pathway",
  "gene_symbol": "NTF3",
  "term_id": "GO:0038180",
  "gene_name": "Neurotrophin-3"
}